{
  "term_id": "GO:0000981",
  "gene_symbol": "ZNF367",
  "gene": "UniProtKB:Q7RTV3",
  "term_label": "DNA-binding transcription factor activity, RNA polymerase II-specific",
  "gene_name": "Zinc finger protein 367"
}